flavonol-3-O-beta-glucoside O-malonyltransferase activity [GO:0047165] (molecular function) Sources: EC:2.3.1.116, MetaCyc:2.3.1.116-RXN Also known as: MAT-3, flavonol 3-O-glucoside malonyltransferase activity, malonyl-CoA:flavonol-3-O-beta-D-glucoside 6''-O-malonyltransferase activity, malonyl-coenzyme A:flavonol-3-O-glucoside malonyltransferase activity Definition: Catalysis of the reaction: flavonol 3-O-beta-D-glucoside + malonyl-CoA = malonyl-flavonol 3-O-beta-D-glucoside + CoA. Relationships: is a type of O-malonyltransferase activity [GO:0050736]